{
  "term_label": "ATP hydrolysis activity",
  "gene_symbol": "KIF2B",
  "term_id": "GO:0016887",
  "gene_name": "Kinesin-like protein KIF2B",
  "gene": "UniProtKB:Q8N4N8"
}